glycine betaine biosynthetic process from glycine [GO:0019286] (biological process) Relationships: is a type of glycine metabolic process [GO:0006544]; is a type of GO:0031456 Sources: GOC:go_curators Definition: The chemical reactions and pathways resulting in the formation of glycine betaine from other compounds, including glycine. Also known as: N-trimethylglycine biosynthesis from glycine, N-trimethylglycine biosynthetic process from glycine, glycine betaine anabolism from glycine, glycine betaine formation from glycine, glycine betaine synthesis from glycine